{
  "gene_name": "ER membrane protein complex subunit 7",
  "term_label": "Unknown molecular function",
  "gene": "UniProtKB:Q9NPA0",
  "term_id": "UNKNOWN:0001",
  "gene_symbol": "EMC7"
}